endoplasmic reticulum [GO:0005783] (CC) Relationships: is a type of GO:0043231; is part of cytoplasm [GO:0005737]; is part of endomembrane system [GO:0012505] Definition: The irregular network of unit membranes, visible only by electron microscopy, that occurs in the cytoplasm of many eukaryotic cells. The membranes form a complex meshwork of tubular channels, which are often expanded into slitlike cavities called cisternae. The ER takes two forms, rough (or granular), with ribosomes adhering to the outer surface, and smooth (with no ribosomes attached). Sources: ISBN:0198506732 Also known as: ER Subtypes: GO:0005790, rough endoplasmic reticulum [GO:0005791], plasmodesmatal endoplasmic reticulum [GO:0009511], sarcoplasmic reticulum [GO:0016529], membrane stack [GO:1990007]